{
  "gene": "UniProtKB:A0A8V8TII8",
  "gene_symbol": "A0A8V8TII8",
  "term_id": "UNKNOWN:0002",
  "gene_name": "Uncharacterized protein",
  "term_label": "Unknown biological process"
}